poly(3-hydroxyalkanoate) biosynthetic process [GO:0042621] (biological process) Also known as: PHA biosynthesis, PHA biosynthetic process, poly(3-hydroxyalkanoate) anabolism, poly(3-hydroxyalkanoate) biosynthesis, poly(3-hydroxyalkanoate) formation, poly(3-hydroxyalkanoate) synthesis Definition: The chemical reactions and pathways resulting in the formation of poly(3-hydroxyalkanoates), polyesters of 3-hydroxyacids produced as intracellular granules by a large variety of bacteria. References: PMID:9925580 Sources: GOC:jl Relationships: is a type of biosynthetic process [GO:0009058]; is a type of poly(3-hydroxyalkanoate) metabolic process [GO:0042620] Regulation: regulated by regulation of poly(3-hydroxyalkanoate) biosynthetic process [GO:0043286]